positive regulation of T cell chemotaxis [GO:0010820] (biological process) Relationships: is a type of regulation of T cell chemotaxis [GO:0010819]; is a type of positive regulation of lymphocyte chemotaxis [GO:0140131]; is a type of GO:2000406; positively regulates T cell chemotaxis [GO:0010818] Sources: GOC:BHF, GOC:dph, GOC:tb Definition: Any process that increases the rate, frequency or extent of T cell chemotaxis. T cell chemotaxis is the directed movement of a T cell in response to an external stimulus.